{
  "term_id": "GO:0042412",
  "gene_symbol": "FMO1",
  "gene_name": "Flavin-containing monooxygenase 1",
  "gene": "UniProtKB:Q01740",
  "term_label": "taurine biosynthetic process"
}